{
  "term_id": "GO:0005667",
  "gene_symbol": "ZFP42",
  "term_label": "transcription regulator complex",
  "gene_name": "Zinc finger protein 42 homolog",
  "gene": "UniProtKB:Q96MM3"
}